{
  "gene_name": "Tumor necrosis factor ligand superfamily member 13",
  "term_id": "GO:0002260",
  "term_label": "lymphocyte homeostasis",
  "gene_symbol": "TNFSF13",
  "gene": "UniProtKB:O75888"
}